{
  "term_id": "GO:0046488",
  "gene_name": "1-phosphatidylinositol 4,5-bisphosphate phosphodiesterase gamma-2",
  "term_label": "phosphatidylinositol metabolic process",
  "gene": "UniProtKB:P16885",
  "gene_symbol": "PLCG2"
}